{
  "term_label": "serine-type endopeptidase inhibitor activity",
  "gene_name": "Protein WFDC11",
  "gene": "UniProtKB:Q8NEX6",
  "term_id": "GO:0004867",
  "gene_symbol": "WFDC11"
}